ABC-type guanine transporter activity [GO:0008558] (molecular function) Definition: Catalyses the reaction: ATP + H2O + guanine(out) = ADP + phosphate + guanine(in). Sources: RHEA:20832 Relationships: is a type of guanine transmembrane transporter activity [GO:0015208]; is a type of GO:0140359 Also known as: guanine ABC transporter, ATP-dependent guanine transmembrane transporter activity, ATPase-coupled guanine transmembrane transporter activity, guanine-transporting ATPase activity